spermatid development [GO:0007286] (biological process) Also known as: spermatid cell development, spermiogenesis Sources: GOC:dph, GOC:go_curators Relationships: is a type of germ cell development [GO:0007281]; is part of spermatid differentiation [GO:0048515] Definition: The process whose specific outcome is the progression of a spermatid over time, from its formation to the mature structure.